tetrahydrofolyl-poly(glutamate) polymer binding [GO:1904493] (molecular function) Definition: Binding to tetrahydrofolyl-poly(glutamate) polymer. Relationships: is a type of small molecule binding [GO:0036094] References: PMID:24863754 Sources: GOC:BHF, GOC:TermGenie, GOC:hal, GO_REF:0000067